{
  "term_label": "Unknown cellular component",
  "gene_name": "Mucosal addressin cell adhesion molecule 1",
  "gene": "UniProtKB:Q13477",
  "gene_symbol": "MADCAM1",
  "term_id": "UNKNOWN:0003"
}